secondary cell wall cellulose synthase complex [GO:0044568] (cellular component) Relationships: is a type of cellulose synthase complex [GO:0010330] Also known as: secondary cell wall CESA complex, secondary cell-wall cellulose synthase complex Definition: A large, multimeric protein complex which catalyzes the biosynthesis of cellulose for the plant secondary cell wall. In Arabidopsis, contains the essential component proteins CESA8, CESA7, and CESA4. References: PMID:21307367 Sources: GOC:mengo_curators, GOC:tt